amino acid catabolic process [GO:0009063] (biological process) Relationships: is a type of GO:0006520; is a type of GO:0009056 Definition: The chemical reactions and pathways resulting in the breakdown of amino acids, organic acids containing one or more amino substituents. Sources: GOC:ai Subtypes: GO:0000955, branched-chain amino acid catabolic process [GO:0009083], GO:0009450, beta-alanine catabolic process [GO:0019484], anaerobic amino acid catabolic process [GO:0019665], nicotianamine catabolic process [GO:0030419], alpha-amino acid catabolic process [GO:1901606] Also known as: amino acid breakdown, amino acid catabolism, amino acid degradation, cellular amino acid catabolic process